{
  "gene_name": "Neurofascin",
  "term_id": "GO:0030424",
  "gene": "UniProtKB:O94856",
  "gene_symbol": "NFASC",
  "term_label": "axon"
}